{
  "term_label": "Unknown cellular component",
  "term_id": "UNKNOWN:0003",
  "gene_name": "Adipocyte plasma membrane-associated protein",
  "gene": "UniProtKB:Q9HDC9",
  "gene_symbol": "APMAP"
}